facial nucleus development [GO:0021754] (biological process) Sources: GOC:cls, GOC:curators, GOC:dgh, GOC:dph, GOC:jid Relationships: is a type of neural nucleus development [GO:0048857]; BFO_0000050 pons development [GO:0021548] Definition: The process whose specific outcome is the progression of the facial nucleus over time, from its formation to the mature structure.